sarcinapterin metabolic process [GO:1900867] (biological process) Sources: GOC:TermGenie, GOC:mengo_curators Definition: The chemical reactions and pathways involving sarcinapterin. Relationships: is a type of phosphate-containing compound metabolic process [GO:0006796]; is a type of organophosphate metabolic process [GO:0019637]; is a type of pteridine-containing compound metabolic process [GO:0042558]; is_a GO:0072350 Subtypes: sarcinapterin biosynthetic process [GO:1900868] Also known as: sarcinapterin metabolism